{
  "term_label": "mRNA binding",
  "gene_name": "Polymerase delta-interacting protein 3",
  "term_id": "GO:0003729",
  "gene_symbol": "POLDIP3",
  "gene": "UniProtKB:Q9BY77"
}